meiotic prometaphase I [GO:0098768] (biological process) Note: This term should not be used for direct annotation. If you are trying to make an annotation to x phase, it is likely that the correct annotation should be to 'regulation of x/y phase transition' or to a process which occurs during the reported phase (e.g. mitotic DNA replication for mitotic S-phase). To capture the phase when a specific location or process is observed, the phase term can be used in an annotation extension (PMID:24885854) applied to a cellular component term (with the relation exists_during) or a biological process term (with the relation happens_during). Relationships: is_a meiosis I cell cycle phase [GO:0098764]; BFO_0000050 meiotic M phase [GO:0051327] References: PMID:16012859 Definition: The meiotic cell cycle phase in eukaryotes between meiotic prophase I and meiotic metaphase I. During meiotic prometaphase I, the nuclear envelope breaks down and one kinetochore forms per chromosome. Chromosomes attach to spindle microtubules and begin to move towards the metaphase plate.